{
  "gene": "UniProtKB:Q9NQ25",
  "term_id": "GO:0006955",
  "gene_symbol": "SLAMF7",
  "term_label": "immune response",
  "gene_name": "SLAM family member 7"
}